{
  "gene_symbol": "YAP1",
  "gene_name": "Transcriptional coactivator YAP1",
  "gene": "UniProtKB:P46937",
  "term_id": "GO:0072091",
  "term_label": "regulation of stem cell proliferation"
}